{
  "term_label": "nucleus",
  "term_id": "GO:0005634",
  "gene": "UniProtKB:Q9NZH4",
  "gene_symbol": "PTTG3P",
  "gene_name": "Putative pituitary tumor-transforming gene 3 protein"
}